{
  "term_id": "GO:0008700",
  "gene_name": "4-hydroxy-2-oxoglutarate aldolase, mitochondrial",
  "gene": "UniProtKB:Q86XE5",
  "term_label": "(R,S)-4-hydroxy-2-oxoglutarate aldolase activity",
  "gene_symbol": "HOGA1"
}